{
  "term_id": "GO:0005669",
  "term_label": "transcription factor TFIID complex",
  "gene_symbol": "TAF9B",
  "gene_name": "Transcription initiation factor TFIID subunit 9B",
  "gene": "UniProtKB:Q9HBM6"
}